{
  "gene_symbol": "NOP14",
  "gene": "UniProtKB:P78316",
  "term_label": "Noc4p-Nop14p complex",
  "term_id": "GO:0030692",
  "gene_name": "Nucleolar protein 14"
}